{
  "gene_name": "Melanoma-associated antigen E2",
  "gene_symbol": "MAGEE2",
  "term_id": "GO:0005634",
  "term_label": "nucleus",
  "gene": "UniProtKB:Q8TD90"
}